{
  "gene_symbol": "CD226",
  "term_label": "positive regulation of immunoglobulin mediated immune response",
  "gene_name": "CD226 antigen",
  "gene": "UniProtKB:Q15762",
  "term_id": "GO:0002891"
}